{
  "gene": "UniProtKB:Q6ZRV3",
  "term_label": "Unknown molecular function",
  "gene_symbol": "LINC00696",
  "term_id": "UNKNOWN:0001",
  "gene_name": "Putative uncharacterized protein encoded by LINC00696"
}